{
  "gene_name": "Protein S100-B",
  "gene_symbol": "S100B",
  "term_id": "GO:0005737",
  "term_label": "cytoplasm",
  "gene": "UniProtKB:P04271"
}